{
  "gene": "UniProtKB:Q99720",
  "gene_name": "Sigma non-opioid intracellular receptor 1",
  "gene_symbol": "SIGMAR1",
  "term_label": "endoplasmic reticulum",
  "term_id": "GO:0005783"
}